{
  "gene_name": "WD repeat-containing protein 1",
  "term_id": "GO:0045214",
  "gene_symbol": "WDR1",
  "gene": "UniProtKB:O75083",
  "term_label": "sarcomere organization"
}